biliverdin reductase [NAD(P)H] activity [GO:0004074] (molecular function) Also known as: biliverdin reductase [NAD(P)+] activity, bilirubin:NAD(P)+ oxidoreductase activity Relationships: is a type of oxidoreductase activity, acting on the CH-CH group of donors, NAD or NADP as acceptor [GO:0016628] Subtypes: GO:0106276, biliverdin reductase (NADPH) activity [GO:0106277] Definition: Catalysis of the reaction: bilirubin IXalpha + NAD(P)+ = biliverdin IXalpha + NAD(P)H + H+. Sources: EC:1.3.1.24